{
  "gene": "UniProtKB:Q6ZRI8",
  "term_label": "GTPase activator activity",
  "term_id": "GO:0005096",
  "gene_name": "Rho GTPase-activating protein 36",
  "gene_symbol": "ARHGAP36"
}